{
  "term_label": "Unknown cellular component",
  "gene_symbol": "PBOV1",
  "gene_name": "Prostate and breast cancer overexpressed gene 1 protein",
  "term_id": "UNKNOWN:0003",
  "gene": "UniProtKB:Q9GZY1"
}